{
  "gene_symbol": "RFX8",
  "term_id": "GO:0000978",
  "gene_name": "DNA-binding protein RFX8",
  "gene": "UniProtKB:Q6ZV50",
  "term_label": "RNA polymerase II cis-regulatory region sequence-specific DNA binding"
}